{
  "gene_symbol": "PAFAH1B1",
  "gene": "UniProtKB:P43034",
  "term_label": "cytoplasmic microtubule",
  "term_id": "GO:0005881",
  "gene_name": "Platelet-activating factor acetylhydrolase IB subunit beta"
}